{
  "term_label": "perinuclear region of cytoplasm",
  "gene_name": "Protein S100-A14",
  "gene": "UniProtKB:Q9HCY8",
  "gene_symbol": "S100A14",
  "term_id": "GO:0048471"
}